{
  "gene_symbol": "RAC3",
  "term_label": "cytoplasmic vesicle",
  "gene_name": "Ras-related C3 botulinum toxin substrate 3",
  "term_id": "GO:0031410",
  "gene": "UniProtKB:P60763"
}